{
  "gene_name": "Dynein light chain Tctex-type 1",
  "gene_symbol": "DYNLT1",
  "gene": "UniProtKB:P63172",
  "term_id": "GO:0005737",
  "term_label": "cytoplasm"
}